positive regulation of mRNA processing [GO:0050685] (biological process) Also known as: up regulation of mRNA processing, up-regulation of mRNA processing, upregulation of mRNA processing, activation of mRNA processing, stimulation of mRNA processing Definition: Any process that activates or increases the frequency, rate or extent of mRNA processing. Sources: GOC:ai Relationships: is a type of GO:0050684; is a type of positive regulation of mRNA metabolic process [GO:1903313]; positively regulates mRNA processing [GO:0006397] Subtypes: positive regulation of mRNA 3'-end processing [GO:0031442], positive regulation of mRNA splicing, via spliceosome [GO:0048026], GO:0160199